{
  "gene_symbol": "PER3",
  "term_id": "GO:0000976",
  "term_label": "transcription cis-regulatory region binding",
  "gene": "UniProtKB:P56645",
  "gene_name": "Period circadian protein homolog 3"
}